{
  "term_label": "Unknown molecular function",
  "term_id": "UNKNOWN:0001",
  "gene_symbol": "PNRC1",
  "gene_name": "Proline-rich nuclear receptor coactivator 1",
  "gene": "UniProtKB:Q12796"
}